{
  "gene": "UniProtKB:P61236",
  "gene_name": "Protein yippee-like 3",
  "term_id": "UNKNOWN:0003",
  "term_label": "Unknown cellular component",
  "gene_symbol": "YPEL3"
}